guanyl nucleotide binding [GO:0019001] (molecular function) Definition: Binding to a guanyl nucleotide, consisting of guanosine esterified with (ortho)phosphate. Subtypes: guanyl deoxyribonucleotide binding [GO:0032560], guanyl ribonucleotide binding [GO:0032561] Sources: ISBN:0198506732 Relationships: is a type of GO:0017076